{
  "term_id": "GO:0006357",
  "gene_name": "Netrin-3",
  "term_label": "regulation of transcription by RNA polymerase II",
  "gene": "UniProtKB:O00634",
  "gene_symbol": "NTN3"
}